negative regulation of galactoglucomannan catabolic process [GO:2000913] (biological process) Definition: Any process that stops, prevents or reduces the frequency, rate or extent of galactoglucomannan catabolic process. Relationships: is a type of negative regulation of catabolic process [GO:0009895]; is a type of negative regulation of macromolecule metabolic process [GO:0010605]; is a type of negative regulation of carbohydrate metabolic process [GO:0045912]; is_a regulation of galactoglucomannan catabolic process [GO:2000912]; negatively regulates galactoglucomannan catabolic process [GO:2000885] Also known as: negative regulation of galactoglucomannan catabolism Sources: GOC:mengo_curators